{
  "gene_symbol": "OFD1",
  "term_label": "Unknown molecular function",
  "gene_name": "Centriole and centriolar satellite protein OFD1",
  "gene": "UniProtKB:O75665",
  "term_id": "UNKNOWN:0001"
}